{
  "gene_name": "Late cornified envelope protein 2C",
  "gene": "UniProtKB:Q5TA81",
  "term_id": "UNKNOWN:0001",
  "term_label": "Unknown molecular function",
  "gene_symbol": "LCE2C"
}